{
  "gene": "UniProtKB:Q9UJ04",
  "term_id": "UNKNOWN:0002",
  "gene_symbol": "TSPYL4",
  "gene_name": "Testis-specific Y-encoded-like protein 4",
  "term_label": "Unknown biological process"
}